regulation of paraxial mesodermal cell fate specification [GO:0048349] (biological process) Definition: Any process that modulates the frequency, rate or extent of paraxial mesoderm cell fate specification. Relationships: is a type of regulation of mesodermal cell fate specification [GO:0042661]; regulates paraxial mesodermal cell fate specification [GO:0048348] Subtypes: GO:0048350, GO:0048351 Sources: GOC:dgh